{
  "term_id": "GO:0022857",
  "gene_symbol": "SLC44A2",
  "gene": "UniProtKB:Q8IWA5",
  "gene_name": "Choline transporter-like protein 2",
  "term_label": "transmembrane transporter activity"
}